{
  "gene_symbol": "ZNF705EP",
  "gene_name": "Putative zinc finger protein 705EP",
  "term_label": "nucleus",
  "term_id": "GO:0005634",
  "gene": "UniProtKB:A8MWA4"
}